{
  "gene": "UniProtKB:Q12907",
  "gene_name": "Vesicular integral-membrane protein VIP36",
  "term_label": "Golgi membrane",
  "gene_symbol": "LMAN2",
  "term_id": "GO:0000139"
}